{
  "gene_symbol": "GSK3B",
  "term_id": "GO:0008013",
  "gene_name": "Glycogen synthase kinase-3 beta",
  "term_label": "beta-catenin binding",
  "gene": "UniProtKB:P49841"
}